{
  "term_id": "GO:0005871",
  "gene_name": "Kinesin-like protein KIF18B",
  "gene_symbol": "KIF18B",
  "gene": "UniProtKB:Q86Y91",
  "term_label": "kinesin complex"
}